transepithelial transport [GO:0070633] (biological process) Subtypes: transepithelial chloride transport [GO:0030321], epithelial fluid transport [GO:0042045], transepithelial ammonium transport [GO:0070634] Regulation: regulated by regulation of transepithelial transport [GO:0150111] Definition: The directed movement of a substance from one side of an epithelium to the other. Relationships: is a type of transport [GO:0006810] Sources: GOC:mah, GOC:yaf, ISBN:0716731363